{
  "gene_name": "Gamma-secretase subunit APH-1B",
  "term_id": "GO:0030674",
  "gene_symbol": "APH1B",
  "term_label": "protein-macromolecule adaptor activity",
  "gene": "UniProtKB:Q8WW43"
}